{
  "term_id": "GO:0004888",
  "term_label": "transmembrane signaling receptor activity",
  "gene_symbol": "ANTXR2",
  "gene_name": "Anthrax toxin receptor 2",
  "gene": "UniProtKB:P58335"
}